sodium-transporting ATP synthase activity, rotational mechanism [GO:0046932] (molecular function) Also known as: sodium-translocating F-type ATPase activity, sodium-transporting two-sector ATPase activity Definition: Enables the transfer of a solute or solutes from one side of a membrane to the other by a rotational mechanism according to the reaction: 4 Na+(out) + ADP + phosphate + H+ => 4 Na+(in) + ATP + H2O. Sources: RHEA:58158 Relationships: is a type of sodium ion transmembrane transporter activity [GO:0015081]; is_a GO:0016874